{
  "gene_symbol": "FXYD4",
  "term_label": "Unknown cellular component",
  "term_id": "UNKNOWN:0003",
  "gene": "UniProtKB:P59646",
  "gene_name": "FXYD domain-containing ion transport regulator 4"
}